{
  "term_label": "plasma membrane",
  "term_id": "GO:0005886",
  "gene_symbol": "ATP1A2",
  "gene": "UniProtKB:P50993",
  "gene_name": "Sodium_potassium-transporting ATPase subunit alpha-2"
}